{
  "gene_symbol": "ZNF44",
  "term_id": "GO:0000981",
  "gene": "UniProtKB:P15621",
  "gene_name": "Zinc finger protein 44",
  "term_label": "DNA-binding transcription factor activity, RNA polymerase II-specific"
}